{
  "term_id": "GO:0005634",
  "gene_symbol": "DMRTA1",
  "term_label": "nucleus",
  "gene_name": "Doublesex- and mab-3-related transcription factor A1",
  "gene": "UniProtKB:Q5VZB9"
}